{
  "gene": "UniProtKB:P19113",
  "gene_symbol": "HDC",
  "term_label": "cytoplasm",
  "gene_name": "Histidine decarboxylase",
  "term_id": "GO:0005737"
}